{
  "gene": "UniProtKB:Q9BZZ5",
  "term_label": "RNA binding",
  "gene_symbol": "API5",
  "term_id": "GO:0003723",
  "gene_name": "Apoptosis inhibitor 5"
}